adaptive immune response based on somatic recombination of immune receptors built from immunoglobulin superfamily domains [GO:0002460] (biological process) Regulation: regulated by regulation of adaptive immune response based on somatic recombination of immune receptors built from immunoglobulin superfamily domains [GO:0002822]; negatively regulated by negative regulation of adaptive immune response based on somatic recombination of immune receptors built from immunoglobulin superfamily domains [GO:0002823]; positively regulated by positive regulation of adaptive immune response based on somatic recombination of immune receptors built from immunoglobulin superfamily domains [GO:0002824] Subtypes: T cell mediated immunity [GO:0002456], tolerance induction dependent upon immune response [GO:0002461], germinal center formation [GO:0002467], B cell mediated immunity [GO:0019724], GO:0042088, GO:0072538, GO:0090717, adaptive immune effector response involving T cells and B lineage cells [GO:0090719], GO:0090721 Relationships: is a type of adaptive immune response [GO:0002250] Sources: GOC:add, GOC:mtg_sensu, ISBN:0781735149, ISBN:1405196831 Definition: An immune response mediated by lymphocytes expressing specific receptors for antigen produced through a somatic diversification process that includes somatic recombination of germline gene segments encoding immunoglobulin superfamily domains. Recombined receptors for antigen encoded by immunoglobulin superfamily domains include T cell receptors and immunoglobulins (antibodies) produced by B cells. The first encounter with antigen elicits a primary immune response that is slow and not of great magnitude. T and B cells selected by antigen become activated and undergo clonal expansion. A fraction of antigen-reactive T and B cells become memory cells, whereas others differentiate into effector cells. The memory cells generated during the primary response enable a much faster and stronger secondary immune response upon subsequent exposures to the same antigen (immunological memory). An example of this is the adaptive immune response found in Mus musculus.